glucosylceramidase activity [GO:0004348] (molecular function) Relationships: is a type of glycosylceramidase activity [GO:0017042] Sources: EC:3.2.1.45 Also known as: D-glucosyl-N-acylsphingosine glucohydrolase activity, GlcCer-beta-glucosidase activity, acid beta-glucosidase activity, beta-D-glucocerebrosidase activity, beta-glucocerebrosidase activity, beta-glucosylceramidase activity, ceramide glucosidase activity, glucocerebrosidase activity, glucosphingosine glucosylhydrolase activity, glucosylcerebrosidase activity, glucosylsphingosine beta-D-glucosidase activity, glucosylsphingosine beta-glucosidase activity, psychosine hydrolase activity Definition: Catalysis of the reaction: D-glucosyl-N-acylsphingosine + H2O = D-glucose + N-acylsphingosine.